{
  "term_label": "Unknown biological process",
  "gene": "UniProtKB:Q96NR7",
  "gene_name": "Putative uncharacterized protein WWC2-AS2",
  "term_id": "UNKNOWN:0002",
  "gene_symbol": "WWC2-AS2"
}